NADH dehydrogenase (ubiquinone) (non-electrogenic) activity [GO:0120555] (MF) Definition: Catalysis of the reaction: a ubiquinone + NADH + H+ = a ubiquinol + NAD+. Sources: RHEA:23152 Relationships: is a type of NADH dehydrogenase (quinone) (non-electrogenic) activity [GO:0050136]